{
  "term_label": "nucleus",
  "gene_name": "Carnosine N-methyltransferase",
  "gene_symbol": "CARNMT1",
  "term_id": "GO:0005634",
  "gene": "UniProtKB:Q8N4J0"
}